negative regulation of gamma-delta T cell proliferation [GO:0046647] (biological process) Relationships: is a type of negative regulation of T cell proliferation [GO:0042130]; is_a negative regulation of gamma-delta T cell activation [GO:0046644]; is a type of regulation of gamma-delta T cell proliferation [GO:0046646]; negatively regulates gamma-delta T cell proliferation [GO:0046630] Sources: GOC:ai Also known as: down regulation of gamma-delta T cell proliferation, down-regulation of gamma-delta T cell proliferation, downregulation of gamma-delta T cell proliferation, negative regulation of gamma-delta T lymphocyte proliferation, negative regulation of gamma-delta T-cell proliferation, negative regulation of gamma-delta T-lymphocyte proliferation, inhibition of gamma-delta T cell proliferation Definition: Any process that stops, prevents, or reduces the frequency, rate or extent of gamma-delta T cell proliferation.